{
  "gene": "UniProtKB:P05107",
  "gene_name": "Integrin beta-2",
  "term_id": "GO:0005925",
  "gene_symbol": "ITGB2",
  "term_label": "focal adhesion"
}